{
  "gene_symbol": "AHR",
  "term_label": "transcription cis-regulatory region binding",
  "gene": "UniProtKB:P35869",
  "gene_name": "Aryl hydrocarbon receptor",
  "term_id": "GO:0000976"
}